nuclear origin of replication recognition complex [GO:0005664] (cellular component) Relationships: is a type of origin recognition complex [GO:0000808]; is a type of nuclear protein-containing complex [GO:0140513]; is part of nuclear chromosome [GO:0000228] Sources: GOC:elh Also known as: eukaryotic ORC, nuclear ORC Definition: A multisubunit complex that is located at the replication origins of a chromosome in the nucleus.